{
  "term_label": "centrosome cycle",
  "gene_name": "Rootletin",
  "term_id": "GO:0007098",
  "gene": "UniProtKB:Q5TZA2",
  "gene_symbol": "CROCC"
}